{
  "gene_name": "Nuclear speckle splicing regulatory protein 1",
  "term_label": "Unknown molecular function",
  "gene_symbol": "NSRP1",
  "term_id": "UNKNOWN:0001",
  "gene": "UniProtKB:Q9H0G5"
}